ornithine carbamoyltransferase inhibitor activity [GO:0090369] (molecular function) Definition: Binds to and stops, prevents, or reduces the activity of ornithine carbamoyltransferase. Sources: GOC:dph, GOC:jp, GOC:tb Relationships: is a type of GO:0004857; negatively regulates ornithine carbamoyltransferase activity [GO:0004585]